inositol diphosphate pentakisphosphate diphosphatase activity [GO:0052842] (molecular function) Subtypes: inositol-1-diphosphate-2,3,4,5,6-pentakisphosphate diphosphatase activity [GO:0052843], inositol-3-diphosphate-1,2,4,5,6-pentakisphosphate diphosphatase activity [GO:0052844], inositol-5-diphosphate-1,2,3,4,6-pentakisphosphate diphosphatase activity [GO:0052845] References: PMID:10827188, PMID:11502751 Relationships: is a type of diphosphoinositol-polyphosphate diphosphatase activity [GO:0008486] Definition: Catalysis of the reaction: diphospho-1D-myo-inositol pentakisphosphate + H2O = 1D-myo-inositol hexakisphosphate + phosphate.